{
  "gene_symbol": "EFNA4",
  "gene": "UniProtKB:P52798",
  "term_label": "axon guidance",
  "gene_name": "Ephrin-A4",
  "term_id": "GO:0007411"
}